{
  "term_label": "Unknown biological process",
  "gene_symbol": "TCF25",
  "gene": "UniProtKB:Q9BQ70",
  "gene_name": "Ribosome quality control complex subunit TCF25",
  "term_id": "UNKNOWN:0002"
}